cellular response to morphine [GO:0071315] (biological process) Sources: GOC:mah Relationships: is a type of response to morphine [GO:0043278]; is a type of cellular response to isoquinoline alkaloid [GO:0071317] Definition: Any process that results in a change in state or activity of a cell (in terms of movement, secretion, enzyme production, gene expression, etc.) as a result of a morphine stimulus. Morphine is an opioid alkaloid, isolated from opium, with a complex ring structure.